{
  "term_label": "Unknown molecular function",
  "gene_symbol": "MAVS",
  "gene_name": "Mitochondrial antiviral-signaling protein",
  "gene": "UniProtKB:Q7Z434",
  "term_id": "UNKNOWN:0001"
}